{
  "term_id": "UNKNOWN:0002",
  "gene": "UniProtKB:A2RUQ5",
  "gene_symbol": "TMEM132E-DT",
  "term_label": "Unknown biological process",
  "gene_name": "Uncharacterized protein TMEM132E-DT"
}